{
  "gene": "UniProtKB:P0CG30",
  "term_label": "cytoplasm",
  "gene_symbol": "GSTT2B",
  "gene_name": "Glutathione S-transferase theta-2B",
  "term_id": "GO:0005737"
}